{
  "gene": "UniProtKB:Q14184",
  "term_label": "synapse",
  "gene_symbol": "DOC2B",
  "gene_name": "Double C2-like domain-containing protein beta",
  "term_id": "GO:0045202"
}